{
  "gene_symbol": "SCNN1B",
  "term_label": "sodium ion transmembrane transport",
  "gene_name": "Amiloride-sensitive sodium channel subunit beta",
  "term_id": "GO:0035725",
  "gene": "UniProtKB:P51168"
}